detection of electrical stimulus involved in regulation of muscle adaptation [GO:0014879] (biological process) Definition: The series of events by which an electrical stimulus is received and converted into a molecular signal. This occurs as part of the regulation of muscle adaptation. Relationships: is a type of response to electrical stimulus involved in regulation of muscle adaptation [GO:0014878]; is a type of detection of electrical stimulus [GO:0050981] Sources: GOC:ef, GOC:mtg_muscle